BBSome [GO:0034464] (cellular component) References: PMID:15231740, PMID:17574030, PMID:26498262 Sources: GOC:BHF, GOC:cilia Relationships: is_a protein-containing complex [GO:0032991]; BFO_0000050 cilium [GO:0005929] Definition: A ciliary protein complex involved in cilium biogenesis. It consists of at least seven Bardet-Biedl syndrome (BBS) proteins and BBIP10. It moves in association with IFT trains through cilia (likely as an IFT-A/B adaptor or cargo), and is required for the integrity of IFT-A and IFT-B. Also known as: Bardet-Biedl syndrome complex